branchiomotor neuron axon guidance [GO:0021785] (biological process) Definition: The process in which a branchiomotor neuron growth cone is directed to a specific target site. Branchiomotor neurons are located in the hindbrain and innervate branchial arch-derived muscles that control jaw movements, facial expression, the larynx, and the pharynx. Subtypes: GO:0021786, branchiomotor neuron axon guidance in branchial arch mesenchyme [GO:0021789] Relationships: is a type of motor neuron axon guidance [GO:0008045] Also known as: BMN axon guidance, branchial motor axon guidance, special visceral motor neuron axon guidance References: PMID:14699587 Sources: GOC:cls, GOC:dgh, GOC:dph, GOC:jid, GO_REF:0000021